{
  "gene_symbol": "RASD1",
  "term_label": "cytoplasm",
  "term_id": "GO:0005737",
  "gene": "UniProtKB:Q9Y272",
  "gene_name": "Dexamethasone-induced Ras-related protein 1"
}